peptidyl-S-diacylglycerol-L-cysteine biosynthetic process from peptidyl-cysteine [GO:0018231] (biological process) Also known as: peptidyl-S-diacylglycerol-L-cysteine anabolism from peptidyl-cysteine, peptidyl-S-diacylglycerol-L-cysteine formation from peptidyl-cysteine, peptidyl-S-diacylglycerol-L-cysteine synthesis from peptidyl-cysteine Relationships: is a type of peptidyl-cysteine modification [GO:0018198] Sources: RESID:AA0107 Definition: The modification of peptidyl-cysteine to form peptidyl-S-diacylglycerol-L-cysteine; the oleate and palmitate actually represent mixtures of saturated (generally at 3') and unsaturated (generally at 2') fatty acids. Subtypes: peptidyl-L-cysteine S-palmitoylation [GO:0018230]